{
  "gene": "UniProtKB:P54105",
  "term_label": "spliceosomal complex",
  "term_id": "GO:0005681",
  "gene_name": "Methylosome subunit pICln",
  "gene_symbol": "CLNS1A"
}